polypeptide N-acetylgalactosaminyltransferase activity [GO:0004653] (molecular function) Relationships: is a type of GO:0008376; is_a GO:0140096 Also known as: UDP-GalNAc:polypeptide N-acetylgalactosaminyl transferase activity, UDP-GalNAc:polypeptide N-acetylgalactosaminyltransferase activity, UDP-N-acetyl-D-galactosamine:polypeptide N-acetylgalactosaminyl-transferase activity, UDP-N-acetyl-alpha-D-galactosamine:polypeptide N-acetylgalactosaminyltransferase activity, UDP-N-acetylgalactosamine-glycoprotein N-acetylgalactosaminyltransferase activity, UDP-N-acetylgalactosamine-protein N-acetylgalactosaminyltransferase activity, UDP-N-acetylgalactosamine:kappa-casein polypeptide N-acetylgalactosaminyltransferase activity, UDP-N-acetylgalactosamine:polypeptide N-acetylgalactosaminyltransferase activity, UDP-N-acetylgalactosamine:protein N-acetylgalactosaminyl transferase activity, UDP-acetylgalactosamine-glycoprotein acetylgalactosaminyltransferase activity, UDP-acetylgalactosamine:peptide-N-galactosaminyltransferase activity, glycoprotein acetylgalactosaminyltransferase activity, polypeptide-N-acetylgalactosamine transferase activity, protein-UDP acetylgalactosaminyltransferase activity, uridine diphosphoacetylgalactosamine-glycoprotein acetylgalactosaminyltransferase activity Definition: Catalysis of the reaction: UDP-N-acetyl-D-galactosamine + polypeptide = UDP + N-acetyl-D-galactosaminyl-polypeptide. This reaction is the modification of serine or threonine residues in polypeptide chains by the transfer of a N-acetylgalactose from UDP-N-acetylgalactose to the hydroxyl group of the amino acid; it is the first step in O-glycan biosynthesis. Sources: EC:2.4.1.41, ISBN:0879695595